{
  "term_id": "GO:0005802",
  "term_label": "trans-Golgi network",
  "gene": "UniProtKB:Q9NZ52",
  "gene_name": "ADP-ribosylation factor-binding protein GGA3",
  "gene_symbol": "GGA3"
}